{
  "gene_symbol": "SLC22A24",
  "gene_name": "Steroid transmembrane transporter SLC22A24",
  "gene": "UniProtKB:Q8N4F4",
  "term_label": "organic anion transport",
  "term_id": "GO:0015711"
}